{
  "gene_name": "Protein transport protein Sec61 subunit alpha isoform 2",
  "gene": "UniProtKB:Q9H9S3",
  "term_label": "ribosome binding",
  "gene_symbol": "SEC61A2",
  "term_id": "GO:0043022"
}